{
  "gene_symbol": "RAB11FIP5",
  "gene": "UniProtKB:Q9BXF6",
  "gene_name": "Rab11 family-interacting protein 5",
  "term_label": "recycling endosome",
  "term_id": "GO:0055037"
}